{
  "term_label": "alpha-tubulin binding",
  "gene_name": "Dynein axonemal light chain 1",
  "gene_symbol": "DNAL1",
  "term_id": "GO:0043014",
  "gene": "UniProtKB:Q4LDG9"
}